{
  "gene_name": "Pulmonary surfactant-associated protein A1",
  "gene_symbol": "SFTPA1",
  "term_id": "UNKNOWN:0001",
  "gene": "UniProtKB:Q8IWL2",
  "term_label": "Unknown molecular function"
}